{
  "gene_name": "Interferon alpha-10",
  "gene_symbol": "IFNA10",
  "term_label": "T cell activation involved in immune response",
  "term_id": "GO:0002286",
  "gene": "UniProtKB:P01566"
}